phosphorus utilization [GO:0006794] (biological process) Definition: A series of processes that forms an integrated mechanism by which a cell or an organism detects the depletion of primary phosphorus source and then activates genes to scavenge the last traces of the primary phosphorus source and to transport and metabolize alternative phosphorus sources. The utilization process begins when the cell or organism detects phosphorus levels, includes the phosphorus-containing substances, and ends when phosphorus is incorporated into the cell or organism's metabolism. Relationships: is a type of phosphorus metabolic process [GO:0006793] Sources: GOC:mah, GOC:mlg Regulation: regulated by regulation of phosphorus utilization [GO:0006795]; negatively regulated by negative regulation of phosphorus utilization [GO:0045942]; positively regulated by GO:0045949